{
  "gene_symbol": "HOOK1",
  "term_id": "GO:0031122",
  "gene_name": "Protein Hook homolog 1",
  "term_label": "cytoplasmic microtubule organization",
  "gene": "UniProtKB:Q9UJC3"
}